plasma membrane of cell tip [GO:0031520] (cellular component) Subtypes: mating projection tip membrane [GO:0070867], plasma membrane of growing cell tip [GO:1902929] Also known as: 'plasma membrane, cell tip' Relationships: is_a plasma membrane region [GO:0098590]; is part of cell tip [GO:0051286] Definition: The portion of the plasma membrane surrounding the cell tip. Sources: GOC:mah